{
  "gene_symbol": "ZNF311",
  "gene": "UniProtKB:Q5JNZ3",
  "term_label": "regulation of transcription by RNA polymerase II",
  "gene_name": "Zinc finger protein 311",
  "term_id": "GO:0006357"
}